{
  "term_id": "GO:0003887",
  "gene_name": "DNA polymerase epsilon catalytic subunit A",
  "gene_symbol": "POLE",
  "term_label": "DNA-directed DNA polymerase activity",
  "gene": "UniProtKB:Q07864"
}